ciliary centrin arm [GO:0120269] (cellular component) Definition: A rod-shaped protein complex containing Centrin4 protein that flanks the flagellum attachment zone (FAZ) filament and the quartet microtubules. References: PMID:26540076, PMID:31217284 Sources: GOC:ach, GOC:krc Note: Note that cilia and eukaryotic flagella are deemed to be equivalent. In diplomonad species, such as Giardia, the axoneme may extend intracellularly up to 5um away from the plane of the plasma membrane. Relationships: is a type of intracellular protein-containing complex [GO:0140535]; is part of ciliary pocket [GO:0020016]